cellular response to N-acetyl-D-glucosamine [GO:0097316] (biological process) Definition: Any process that results in a change in state or activity of a cell (in terms of movement, secretion, enzyme production, gene expression, etc.) as a result of an N-acetyl-D-glucosamine stimulus. References: PMID:21700702 Sources: GOC:di Relationships: is a type of response to N-acetyl-D-glucosamine [GO:0097315]; is a type of GO:1901701